{
  "gene": "UniProtKB:Q02318",
  "gene_name": "Sterol 26-hydroxylase, mitochondrial",
  "gene_symbol": "CYP27A1",
  "term_label": "cholesterol metabolic process",
  "term_id": "GO:0008203"
}